spliceosomal snRNP complex [GO:0097525] (cellular component) Definition: A small ribonucleoprotein complex involved in formation of the spliceosome. Subtypes: U5 snRNP [GO:0005682], GO:0005685, GO:0005686, U4 snRNP [GO:0005687], GO:0005688, U4atac snRNP [GO:0005690], GO:0005691, U11 snRNP [GO:0005692], GO:0005693, U11/U12 snRNP [GO:0034693], U4/U6 snRNP [GO:0071001], GO:0071002, penta-snRNP complex [GO:0071003], SL snRNP [GO:0071024], spliceosomal tri-snRNP complex [GO:0097526] Relationships: is a type of small nuclear ribonucleoprotein complex [GO:0030532] Sources: GOC:krc, GOC:pr, ISBN:0879695897